{
  "gene_name": "Uncharacterized protein C17orf100",
  "gene_symbol": "C17orf100",
  "term_id": "UNKNOWN:0001",
  "gene": "UniProtKB:A8MU93",
  "term_label": "Unknown molecular function"
}